{
  "gene": "UniProtKB:Q5VWC8",
  "term_id": "GO:0042761",
  "term_label": "very long-chain fatty acid biosynthetic process",
  "gene_name": "Very-long-chain (3R)-3-hydroxyacyl-CoA dehydratase 4",
  "gene_symbol": "HACD4"
}